{
  "gene_name": "Potassium voltage-gated channel subfamily S member 2",
  "term_id": "GO:0016020",
  "gene": "UniProtKB:Q9ULS6",
  "gene_symbol": "KCNS2",
  "term_label": "membrane"
}